{
  "term_id": "GO:0009897",
  "gene": "UniProtKB:P51685",
  "gene_name": "C-C chemokine receptor type 8",
  "term_label": "external side of plasma membrane",
  "gene_symbol": "CCR8"
}